{
  "term_label": "copper ion import",
  "gene_name": "Copper-transporting ATPase 1",
  "term_id": "GO:0015677",
  "gene_symbol": "ATP7A",
  "gene": "UniProtKB:Q04656"
}